{
  "term_label": "FAD binding",
  "gene_symbol": "AIFM1",
  "gene": "UniProtKB:O95831",
  "term_id": "GO:0071949",
  "gene_name": "Apoptosis-inducing factor 1, mitochondrial"
}